{
  "gene_symbol": "BLOC1S2",
  "gene": "UniProtKB:Q6QNY1",
  "term_id": "GO:0032418",
  "gene_name": "Biogenesis of lysosome-related organelles complex 1 subunit 2",
  "term_label": "lysosome localization"
}